{
  "gene_symbol": "CHRNA7",
  "term_label": "calcium ion transport",
  "gene_name": "Neuronal acetylcholine receptor subunit alpha-7",
  "gene": "UniProtKB:P36544",
  "term_id": "GO:0006816"
}